{
  "gene_name": "Low affinity immunoglobulin gamma Fc region receptor II-a",
  "gene": "UniProtKB:P12318",
  "gene_symbol": "FCGR2A",
  "term_label": "cell surface receptor signaling pathway",
  "term_id": "GO:0007166"
}